B cell antigen processing and presentation [GO:0002450] (biological process) Definition: The process in which a B cell expresses antigen (peptide or lipid) on its cell surface in association with an MHC protein complex. Also known as: B lymphocyte antigen processing and presentation, B-cell antigen processing and presentation, B-lymphocyte antigen processing and presentation Relationships: is a type of antigen processing and presentation [GO:0019882]; is part of GO:0019724 References: PMID:15771591 Sources: GOC:add, ISBN:0781735149 Regulation: regulated by regulation of B cell antigen processing and presentation [GO:0002622]; negatively regulated by negative regulation of B cell antigen processing and presentation [GO:0002623]; positively regulated by GO:0002624 Subtypes: B cell antigen processing and presentation mediated by B cell receptor uptake of antigen [GO:0002417], B cell antigen processing and presentation following pinocytosis [GO:0002421]